sodium-dependent organic cation transport [GO:0070715] (biological process) Relationships: is_a organic cation transport [GO:0015695] Definition: The directed, sodium-dependent, movement of organic cations into, out of or within a cell, or between cells, by means of some agent such as a transporter or pore. Sources: GOC:BHF, GOC:mah